regulation of cartilage development [GO:0061035] (biological process) Definition: Any process that modulates the rate, frequency, or extent of cartilage development, the process whose specific outcome is the progression of the cartilage over time, from its formation to the mature structure. Cartilage is a connective tissue dominated by extracellular matrix containing collagen type II and large amounts of proteoglycan, particularly chondroitin sulfate. Sources: GOC:dph Relationships: is a type of regulation of multicellular organismal development [GO:2000026]; regulates cartilage development [GO:0051216] Subtypes: regulation of chondrocyte differentiation [GO:0032330], positive regulation of cartilage development [GO:0061036], negative regulation of cartilage development [GO:0061037]